{
  "gene_symbol": "ADCYAP1",
  "term_id": "GO:0032880",
  "term_label": "regulation of protein localization",
  "gene_name": "Pituitary adenylate cyclase-activating polypeptide",
  "gene": "UniProtKB:P18509"
}